{
  "gene": "UniProtKB:Q8WXG6",
  "term_label": "cytosol",
  "gene_name": "MAP kinase-activating death domain protein",
  "term_id": "GO:0005829",
  "gene_symbol": "MADD"
}